negative regulation of mast cell differentiation [GO:0060377] (biological process) Definition: Any process that decreases the rate, frequency or extent of mast cell differentiation, the process in which a relatively unspecialized myeloid precursor cell acquires the specialized features of a mast cell. A mast cell is a cell that is found in almost all tissues containing numerous basophilic granules and capable of releasing large amounts of histamine and heparin upon activation. Sources: GOC:dph, GOC:tb Relationships: is a type of negative regulation of myeloid leukocyte differentiation [GO:0002762]; is a type of regulation of mast cell differentiation [GO:0060375]; negatively regulates GO:0060374